histone H3K23ac reader activity [GO:0140118] (molecular function) Relationships: is a type of histone H3 reader activity [GO:0140006] References: PMID:21164480 Note: Comment: Note that the residue position corresponds to the canonical human H3 histone (UniProtKB:P84243); this residue is conserved across all eukaryotes. Residue 1 is the first residue following removal of the initiating Methionine (Met). Note that each histone is encoded by multiple genes, and sequences may vary across different genes within an organism. Definition: A histone reader that recognizes a histone H3 acetylated at lysine 23. Also known as: histone H3K23ac modified histone binding